{
  "gene": "UniProtKB:P98088",
  "gene_symbol": "MUC5AC",
  "term_label": "Unknown biological process",
  "term_id": "UNKNOWN:0002",
  "gene_name": "Mucin-5AC"
}